{
  "term_id": "UNKNOWN:0001",
  "term_label": "Unknown molecular function",
  "gene_symbol": "SPAG11B",
  "gene_name": "Sperm-associated antigen 11B",
  "gene": "UniProtKB:Q08648"
}